{
  "term_label": "DNA-binding transcription factor activity, RNA polymerase II-specific",
  "gene_symbol": "POU3F2",
  "gene_name": "POU domain, class 3, transcription factor 2",
  "gene": "UniProtKB:P20265",
  "term_id": "GO:0000981"
}